{
  "term_id": "GO:0004930",
  "gene": "UniProtKB:O00254",
  "term_label": "G protein-coupled receptor activity",
  "gene_symbol": "F2RL2",
  "gene_name": "Proteinase-activated receptor 3"
}